{
  "term_label": "Unknown molecular function",
  "gene_name": "Immunoglobulin kappa variable 1-17",
  "gene_symbol": "IGKV1-17",
  "gene": "UniProtKB:P01599",
  "term_id": "UNKNOWN:0001"
}